peptidyl-arginine N-methylation [GO:0035246] (biological process) Subtypes: GO:0035247 Relationships: is a type of peptidyl-arginine methylation [GO:0018216] Definition: The addition of a methyl group onto a nitrogen atom of an arginine residue in a protein. Sources: GOC:bf